{
  "gene": "UniProtKB:Q86UK0",
  "term_label": "lipid transport",
  "gene_symbol": "ABCA12",
  "gene_name": "Glucosylceramide transporter ABCA12",
  "term_id": "GO:0006869"
}